{
  "term_label": "phosphatidylcholine lysophospholipase activity",
  "term_id": "GO:0004622",
  "gene_symbol": "GDPD3",
  "gene": "UniProtKB:Q7L5L3",
  "gene_name": "Lysophospholipase D GDPD3"
}